{
  "term_id": "UNKNOWN:0003",
  "term_label": "Unknown cellular component",
  "gene": "UniProtKB:Q09327",
  "gene_name": "Beta-1,4-mannosyl-glycoprotein 4-beta-N-acetylglucosaminyltransferase",
  "gene_symbol": "MGAT3"
}